{
  "gene": "UniProtKB:Q8NEW0",
  "gene_symbol": "SLC30A7",
  "gene_name": "Zinc transporter 7",
  "term_label": "intracellular zinc ion homeostasis",
  "term_id": "GO:0006882"
}